{
  "gene": "UniProtKB:Q16576",
  "gene_symbol": "RBBP7",
  "gene_name": "Histone-binding protein RBBP7",
  "term_id": "GO:0016581",
  "term_label": "NuRD complex"
}